regulation of presynapse organization [GO:0099174] (biological process) Subtypes: regulation of presynapse assembly [GO:1905606], regulation of terminal button organization [GO:2000331] Definition: Any process that modulates the physical form of a presynapse. Also known as: regulation of presynapse organisation, regulation of presynapse structure, regulation of presynapse organization and biogenesis Relationships: is a type of regulation of synapse organization [GO:0050807]; regulates presynapse organization [GO:0099172] Sources: GOC:ai, GOC:dph, GOC:tb